regulation of vasoconstriction by circulating epinephrine [GO:0003120] (biological process) Definition: Any process that modulates the frequency, rate or extent of reductions in the diameter of blood vessels as a result of secretion of epinephrine into the bloodstream. Relationships: is a type of GO:0003115 Sources: GOC:mtg_cardio Also known as: regulation of vasoconstriction by circulating adrenaline